{
  "term_label": "Unknown molecular function",
  "term_id": "UNKNOWN:0001",
  "gene": "UniProtKB:A6NML5",
  "gene_symbol": "TMEM212",
  "gene_name": "Transmembrane protein 212"
}